isobutyryl-CoA mutase activity [GO:0047727] (molecular function) Relationships: is a type of GO:0016866 Definition: Catalysis of the reaction: isobutyryl-CoA = butanoyl-CoA. Sources: EC:5.4.99.13, RHEA:13141 Also known as: 2-methylpropanoyl-CoA CoA-carbonylmutase activity, butyryl-CoA:isobutyryl-CoA mutase activity, isobutyryl coenzyme A mutase activity